alpha-bisabolene synthase activity [GO:0052681] (MF) Also known as: bisabolene synthase activity, (2E,6E)-farnesyl-diphosphate diphosphate-lyase [(E)-alpha-bisabolene-forming] activity Definition: Catalysis of the reaction: 2-trans,6-trans-farnesyl diphosphate = (E,R)-alpha-bisabolene + diphosphate. Relationships: is a type of carbon-oxygen lyase activity, acting on phosphates [GO:0016838] Sources: RHEA:25436